{
  "term_label": "calcium ion binding",
  "gene_name": "Testican-3",
  "gene": "UniProtKB:Q9BQ16",
  "term_id": "GO:0005509",
  "gene_symbol": "SPOCK3"
}